{
  "gene_name": "Centrosomal protein of 295 kDa",
  "term_label": "centrosome",
  "gene_symbol": "CEP295",
  "term_id": "GO:0005813",
  "gene": "UniProtKB:Q9C0D2"
}